positive regulation of signal transduction by receptor internalization [GO:0038010] (biological process) Subtypes: positive regulation of insulin receptor signaling pathway by insulin receptor internalization [GO:0038015], positive regulation of toll-like receptor 9 signaling pathway by B cell receptor internalization [GO:1901245] Definition: Any process in which the internalization of a signaling receptor activates or increases the frequency, rate or extent of signal transduction. Receptor internalization can enhance signaling by concentrating signaling molecules in one location, or by moving a ligand-activated receptor to the location of downstream signaling proteins. Endosomes for example can serve as important intracellular signaling platforms. Also known as: positive regulation of signaling pathway by receptor endocytosis References: PMID:17908284, PMID:19696798 Sources: GOC:bf, GOC:signaling Relationships: is a type of GO:0009967; is a type of regulation of signal transduction by receptor internalization [GO:0038009]